{
  "gene_symbol": "DMTN",
  "term_id": "GO:0005886",
  "term_label": "plasma membrane",
  "gene": "UniProtKB:Q08495",
  "gene_name": "Dematin"
}